{
  "gene_symbol": "SRC",
  "gene": "UniProtKB:P12931",
  "term_label": "negative regulation of intrinsic apoptotic signaling pathway",
  "term_id": "GO:2001243",
  "gene_name": "Proto-oncogene tyrosine-protein kinase Src"
}